{
  "gene_symbol": "IFNA5",
  "term_label": "response to exogenous dsRNA",
  "gene": "UniProtKB:P01569",
  "term_id": "GO:0043330",
  "gene_name": "Interferon alpha-5"
}